dinoflagellate apical groove [GO:0097685] (cellular component) Definition: A cell surface furrow (or groove) found on a dinoflagellate apex. It typically loops around the apex. Relationships: is a type of cell surface furrow [GO:0097610]; is part of dinoflagellate epicone [GO:0097613] Note: The term name refers to a taxonomic group to make the label unique with respect to similarly-named anatomical structures. References: PMID:20561119 Sources: GOC:at, Wikipedia:Dinoflagellate#Morphology, http://tolweb.org/Dinoflagellates/2445 Also known as: apical groove